{
  "gene": "UniProtKB:Q12950",
  "term_label": "regulation of transcription by RNA polymerase II",
  "gene_name": "Forkhead box protein D4",
  "term_id": "GO:0006357",
  "gene_symbol": "FOXD4"
}